{
  "gene_symbol": "KIF2C",
  "term_id": "GO:0005819",
  "gene_name": "Kinesin-like protein KIF2C",
  "gene": "UniProtKB:Q99661",
  "term_label": "spindle"
}